{
  "gene_symbol": "KLHL30",
  "term_label": "proteasome-mediated ubiquitin-dependent protein catabolic process",
  "term_id": "GO:0043161",
  "gene_name": "Kelch-like protein 30",
  "gene": "UniProtKB:Q0D2K2"
}